{
  "term_label": "mitotic spindle assembly checkpoint signaling",
  "term_id": "GO:0007094",
  "gene": "UniProtKB:O43670",
  "gene_symbol": "ZNF207",
  "gene_name": "BUB3-interacting and GLEBS motif-containing protein ZNF207"
}